{
  "gene_symbol": "DST",
  "term_label": "cytoplasm",
  "gene_name": "Dystonin",
  "term_id": "GO:0005737",
  "gene": "UniProtKB:Q03001"
}